{
  "term_id": "GO:0000978",
  "term_label": "RNA polymerase II cis-regulatory region sequence-specific DNA binding",
  "gene_symbol": "GATA3",
  "gene_name": "Trans-acting T-cell-specific transcription factor GATA-3",
  "gene": "UniProtKB:P23771"
}